2-oxoglutarate decarboxylase activity [GO:0008683] (MF) Also known as: 2-oxoglutarate carboxy-lyase (succinate-semialdehyde-forming), 2-oxoglutarate carboxy-lyase activity, alpha-ketoglutarate decarboxylase activity, alpha-ketoglutaric decarboxylase activity, pre-2-oxoglutarate decarboxylase activity Sources: EC:4.1.1.71, RHEA:10524 Relationships: is a type of carboxy-lyase activity [GO:0016831] Definition: Catalysis of the reaction: 2-oxoglutarate + H+ = CO2 + succinate semialdehyde.